{
  "gene_name": "Sarcosine dehydrogenase, mitochondrial",
  "term_id": "GO:1901053",
  "gene": "UniProtKB:Q9UL12",
  "gene_symbol": "SARDH",
  "term_label": "sarcosine catabolic process"
}